{
  "gene": "UniProtKB:Q9NW07",
  "term_label": "RNA polymerase II cis-regulatory region sequence-specific DNA binding",
  "gene_name": "Zinc finger protein 358",
  "gene_symbol": "ZNF358",
  "term_id": "GO:0000978"
}